T cell mediated immunity [GO:0002456] (biological process) Definition: Any process involved in the carrying out of an immune response by a T cell. Relationships: is a type of lymphocyte mediated immunity [GO:0002449]; is a type of adaptive immune response based on somatic recombination of immune receptors built from immunoglobulin superfamily domains [GO:0002460] Regulation: regulated by regulation of T cell mediated immunity [GO:0002709]; negatively regulated by negative regulation of T cell mediated immunity [GO:0002710]; positively regulated by positive regulation of T cell mediated immunity [GO:0002711] Subtypes: type IV hypersensitivity [GO:0001806], T cell mediated cytotoxicity [GO:0001913], GO:0002369, GO:0002424, peripheral T cell tolerance induction [GO:0002458] Also known as: cell-mediated immunity, cellular immune response, T lymphocyte mediated immunity, T-cell mediated immunity, T-lymphocyte mediated immunity Sources: GOC:add, GO_REF:0000022, ISBN:0781735149